negative chemotaxis [GO:0050919] (biological process) Relationships: is a type of chemotaxis [GO:0006935] Definition: The directed movement of a motile cell or organism towards a lower concentration of a chemical. Subtypes: synaptic target inhibition [GO:0016201], chemorepulsion involved in embryonic olfactory bulb interneuron precursor migration [GO:0021834], chemorepulsion involved in postnatal olfactory bulb interneuron migration [GO:0021836], chemorepulsion involved in interneuron migration from the subpallium to the cortex [GO:0021842], chemorepulsion involved in precerebellar neuron migration [GO:0021950], germ cell repulsion [GO:0035233], negative aerotaxis [GO:0052130], chemorepulsion of axon [GO:0061643] Regulation: regulated by regulation of negative chemotaxis [GO:0050923]; positively regulated by positive regulation of negative chemotaxis [GO:0050924]; negatively regulated by negative regulation of negative chemotaxis [GO:0050925] Sources: GOC:ai, GOC:bf, GOC:isa_complete Also known as: chemoaversion, chemorepulsion